{
  "gene": "UniProtKB:P55268",
  "term_id": "GO:0005201",
  "gene_symbol": "LAMB2",
  "gene_name": "Laminin subunit beta-2",
  "term_label": "extracellular matrix structural constituent"
}